{
  "gene_symbol": "ALDH3A2",
  "gene_name": "Aldehyde dehydrogenase family 3 member A2",
  "gene": "UniProtKB:P51648",
  "term_label": "membrane",
  "term_id": "GO:0016020"
}